{
  "term_id": "GO:0019955",
  "gene_symbol": "IL12RB2",
  "term_label": "cytokine binding",
  "gene": "UniProtKB:Q99665",
  "gene_name": "Interleukin-12 receptor subunit beta-2"
}